{
  "term_id": "GO:0035809",
  "gene_symbol": "ADM5",
  "term_label": "regulation of urine volume",
  "gene_name": "Putative adrenomedullin-5-like protein",
  "gene": "UniProtKB:C9JUS6"
}